{
  "gene_name": "Transmembrane protein 126A",
  "gene": "UniProtKB:Q9H061",
  "gene_symbol": "TMEM126A",
  "term_label": "mitochondrial respiratory chain complex I assembly",
  "term_id": "GO:0032981"
}